T-helper 17 cell chemotaxis [GO:0035705] (biological process) Definition: The directed movement of a T-helper 17 cell in response to an external stimulus. Sources: CL:0000899, GOC:BHF Also known as: Th17 cell chemotaxis Relationships: is a type of T cell chemotaxis [GO:0010818]